{
  "term_label": "regulation of canonical Wnt signaling pathway",
  "gene_symbol": "CCNYL2",
  "gene": "UniProtKB:Q5T2Q4",
  "gene_name": "Cyclin-Y-like protein 2",
  "term_id": "GO:0060828"
}